actin lateral binding [GO:0003786] (molecular function) Sources: GOC:mah Relationships: is_a actin filament binding [GO:0051015] Definition: Binding to an actin filament along its length.